{
  "gene_name": "Group 10 secretory phospholipase A2",
  "gene": "UniProtKB:O15496",
  "gene_symbol": "PLA2G10",
  "term_id": "GO:0047498",
  "term_label": "calcium-dependent phospholipase A2 activity"
}